succinate dehydrogenase activity [GO:0000104] (molecular function) Subtypes: GO:0008177, fumarate reductase (NADH) activity [GO:0016156] Also known as: succinic dehydrogenase activity, fumarate dehydrogenase activity, fumarate reductase activity, succinate oxidoreductase activity, succinic acid dehydrogenase activity, succinodehydrogenase activity, succinyl dehydrogenase activity, fumaric hydrogenase activity Definition: Catalysis of the reaction: succinate + acceptor = fumarate + reduced acceptor. Relationships: is a type of oxidoreductase activity, acting on the CH-CH group of donors [GO:0016627] Sources: RHEA:16357 Regulation: positively regulated by positive regulation of succinate dehydrogenase activity [GO:1904231]